outward rectifier potassium channel activity [GO:0015271] (molecular function) Regulation: negatively regulated by GO:0140628 Definition: Enables the transmembrane transfer of a potassium ion by an outwardly-rectifying voltage-gated channel. An outwardly rectifying current-voltage relation is one where at any given driving force the outward flow of K+ ions exceeds the inward flow for the opposite driving force. Subtypes: GO:0005250 Relationships: is a type of voltage-gated potassium channel activity [GO:0005249] Sources: GOC:mah